bent DNA binding [GO:0003681] (molecular function) Definition: Binding to DNA in a bent conformation. References: PMID:12627977 Sources: GOC:jl Relationships: is a type of GO:0003677